{
  "gene": "UniProtKB:Q8IYK8",
  "gene_symbol": "REM2",
  "gene_name": "GTP-binding protein REM 2",
  "term_id": "GO:0005886",
  "term_label": "plasma membrane"
}